{
  "term_label": "vesicle",
  "gene_symbol": "CST4",
  "gene": "UniProtKB:P01036",
  "gene_name": "Cystatin-S",
  "term_id": "GO:0031982"
}